interleukin-35-mediated signaling pathway [GO:0070757] (biological process) Also known as: IL-35-mediated signaling pathway, interleukin-35-mediated signalling pathway Definition: The series of molecular signals initiated by interleukin-35 binding to its receptor on the surface of a target cell, and ending with the regulation of a downstream cellular process, e.g. transcription. Relationships: is a type of cytokine-mediated signaling pathway [GO:0019221] Sources: GOC:add, GOC:mah, GOC:signaling Regulation: regulated by regulation of interleukin-35-mediated signaling pathway [GO:0070758]; RO_0002212 by negative regulation of interleukin-35-mediated signaling pathway [GO:0070759]; positively regulated by positive regulation of interleukin-35-mediated signaling pathway [GO:0070760]